{
  "gene": "UniProtKB:O43474",
  "gene_symbol": "KLF4",
  "gene_name": "Krueppel-like factor 4",
  "term_label": "nucleus",
  "term_id": "GO:0005634"
}